{
  "gene_name": "Slit homolog 2 protein",
  "gene": "UniProtKB:O94813",
  "term_label": "retinal ganglion cell axon guidance",
  "term_id": "GO:0031290",
  "gene_symbol": "SLIT2"
}